{
  "term_label": "superoxide-generating NAD(P)H oxidase activity",
  "gene_symbol": "DUOX1",
  "gene_name": "Dual oxidase 1",
  "gene": "UniProtKB:Q9NRD9",
  "term_id": "GO:0016175"
}